regulation of pyruvate decarboxylation to acetyl-CoA [GO:0010510] (biological process) Subtypes: positive regulation of pyruvate decarboxylation to acetyl-CoA [GO:0140176], negative regulation of pyruvate decarboxylation to acetyl-CoA [GO:0160218] Also known as: regulation of acetyl-CoA biosynthetic process from pyruvate Sources: GOC:dph, GOC:tb Relationships: is a type of regulation of acyl-CoA biosynthetic process [GO:0050812]; regulates pyruvate decarboxylation to acetyl-CoA [GO:0006086] Definition: Any process that modulates the frequency, rate or extent of the chemical reactions and pathways resulting in the formation of acetyl-CoA from pyruvate. In most organisms, this pathway links glycolysis to the TCA cycle, by a series of three reactions carried out by a multisubunit complex called the 'pyruvate dehydrogenase complex', even though pyruvate dehydrogenase activity describes only one of those reactions.